apiose biosynthetic process [GO:0033350] (biological process) Definition: The chemical reactions and pathways resulting in the formation of apiose, the branched tetrose 3-C-(hydroxymethyl)-D-glycero-tetrose. Sources: GOC:mah Also known as: apiose anabolism, apiose biosynthesis, apiose formation, apiose synthesis Relationships: is a type of tetrose biosynthetic process [GO:0033348]